{
  "term_label": "neuron projection regeneration",
  "gene_symbol": "OMG",
  "gene": "UniProtKB:P23515",
  "gene_name": "Oligodendrocyte-myelin glycoprotein",
  "term_id": "GO:0031102"
}